{
  "gene": "UniProtKB:P60893",
  "term_label": "G protein-coupled receptor activity",
  "term_id": "GO:0004930",
  "gene_symbol": "GPR85",
  "gene_name": "Probable G-protein coupled receptor 85"
}